{
  "gene_symbol": "MAP7D3",
  "gene": "UniProtKB:Q8IWC1",
  "term_label": "Unknown molecular function",
  "gene_name": "MAP7 domain-containing protein 3",
  "term_id": "UNKNOWN:0001"
}